{
  "gene": "UniProtKB:Q15700",
  "term_id": "GO:0035418",
  "gene_symbol": "DLG2",
  "gene_name": "Disks large homolog 2",
  "term_label": "protein localization to synapse"
}